MHC class I protein binding, via lateral surface [GO:0023028] (MF) Definition: Binding to a major histocompatibility complex class I molecules via the lateral surface. Sources: GOC:mtg_signal, GOC:vw Relationships: is a type of MHC class I protein binding [GO:0042288]